symbiont-mediated occlusion of host xylem [GO:0052112] (biological process) Also known as: occlusion by symbiont of host xylem Definition: The process in which an organism reduces the flow of fluid within the host xylem, the tissue in plants that carries water and nutrients up from the roots to the shoot and leaves. The host is defined as the larger of the organisms involved in a symbiotic interaction. References: PMID:28871268 Relationships: is a type of symbiont-mediated disruption of host anatomical structure [GO:0052111]